{
  "gene": "UniProtKB:P04118",
  "gene_name": "Colipase",
  "gene_symbol": "CLPS",
  "term_id": "UNKNOWN:0002",
  "term_label": "Unknown biological process"
}